{
  "gene_symbol": "CSTA",
  "term_label": "cysteine-type endopeptidase inhibitor activity",
  "gene": "UniProtKB:P01040",
  "term_id": "GO:0004869",
  "gene_name": "Cystatin-A"
}